{
  "gene_name": "Sphingosine 1-phosphate receptor 4",
  "term_label": "cytoplasm",
  "term_id": "GO:0005737",
  "gene_symbol": "S1PR4",
  "gene": "UniProtKB:O95977"
}